{
  "gene_symbol": "CARMIL3",
  "term_id": "GO:0034315",
  "gene_name": "Capping protein, Arp2_3 and myosin-I linker protein 3",
  "gene": "UniProtKB:Q8ND23",
  "term_label": "regulation of Arp2/3 complex-mediated actin nucleation"
}